COPI coating of Golgi vesicle, inter-Golgi cisterna [GO:0010787] (biological process) Sources: GOC:dph, GOC:tb Definition: The addition of COPI proteins and adaptor proteins to Golgi membranes during the formation of inter-Golgi cisterna transport vesicles, forming a vesicle coat. Relationships: is a type of COPI coating of Golgi vesicle [GO:0048205]; is part of vesicle targeting, inter-Golgi cisterna [GO:0048204]